{
  "gene_name": "Zinc finger and BTB domain-containing protein 41",
  "term_label": "regulation of transcription by RNA polymerase II",
  "gene": "UniProtKB:Q5SVQ8",
  "term_id": "GO:0006357",
  "gene_symbol": "ZBTB41"
}